{
  "gene_symbol": "ABHD2",
  "term_label": "monoacylglycerol lipase activity",
  "gene_name": "Monoacylglycerol lipase ABHD2",
  "term_id": "GO:0047372",
  "gene": "UniProtKB:P08910"
}